{
  "term_id": "GO:0045165",
  "gene": "UniProtKB:O14905",
  "gene_symbol": "WNT9B",
  "term_label": "cell fate commitment",
  "gene_name": "Protein Wnt-9b"
}